{
  "gene": "UniProtKB:Q9GZR1",
  "term_label": "cytoplasm",
  "term_id": "GO:0005737",
  "gene_name": "Sentrin-specific protease 6",
  "gene_symbol": "SENP6"
}